regulation of cell development [GO:0060284] (biological process) Subtypes: positive regulation of cell development [GO:0010720], GO:0010721, regulation of ascospore formation [GO:0034307], GO:0042478, regulation of skeletal muscle fiber development [GO:0048742], regulation of neurogenesis [GO:0050767], GO:0055018, negative regulation of respiratory burst involved in inflammatory response [GO:0060266], regulation of chondrocyte development [GO:0061181], regulation of metula development [GO:0070802], regulation of phialide development [GO:0070805], GO:0070808, modulation of spore encystment on host [GO:0075215], GO:0075306, regulation of establishment of blood-brain barrier [GO:0090210], regulation of endothelial cell development [GO:1901550], regulation of cell maturation [GO:1903429], regulation of hemopoiesis [GO:1903706], GO:1904444, GO:1905079, GO:1905298, regulation of cardiac myofibril assembly [GO:1905304], regulation of oogenesis [GO:1905879], regulation of type B pancreatic cell development [GO:2000074], regulation of metanephric podocyte development [GO:2000477] Relationships: is a type of regulation of cell differentiation [GO:0045595]; regulates cell development [GO:0048468] Definition: Any process that modulates the rate, frequency or extent of the progression of the cell over time, from its formation to the mature structure. Cell development does not include the steps involved in committing a cell to a specific fate. Sources: GOC:dph, GOC:tb